{
  "gene": "UniProtKB:A0A8I5KW96",
  "gene_symbol": "AK4P3",
  "gene_name": "Adenylate kinase 4, mitochondrial",
  "term_id": "GO:0005737",
  "term_label": "cytoplasm"
}